{
  "term_id": "GO:0044233",
  "gene": "UniProtKB:Q96JX3",
  "term_label": "mitochondria-associated endoplasmic reticulum membrane contact site",
  "gene_name": "Protein SERAC1",
  "gene_symbol": "SERAC1"
}